{
  "gene": "UniProtKB:Q96AG3",
  "gene_name": "Mitochondrial outer membrane protein SLC25A46",
  "gene_symbol": "SLC25A46",
  "term_label": "Unknown molecular function",
  "term_id": "UNKNOWN:0001"
}